{
  "term_label": "very long-chain fatty acid biosynthetic process",
  "term_id": "GO:0042761",
  "gene_name": "Elongation of very long chain fatty acids protein 4",
  "gene": "UniProtKB:Q9GZR5",
  "gene_symbol": "ELOVL4"
}